succinate-semialdehyde dehydrogenase (NADP+) activity [GO:0036243] (molecular function) Sources: GOC:bf, RHEA:13213 Definition: Catalysis of the reaction: succinate semialdehyde + NADP+ + H2O = succinate + NADPH + 2 H+. Relationships: is a type of GO:0009013 Also known as: NADP-dependent succinate-semialdehyde dehydrogenase activity, succinate semialdehyde:NADP+ oxidoreductase activity, succinic semialdehyde dehydrogenase (NADP+) activity, succinyl semialdehyde dehydrogenase (NADP+) activity Note: This function is similar to EC:1.2.1.24 [succinate-semialdehyde dehydrogenase (NAD+)], and EC:1.2.1.16 [succinate-semialdehyde dehydrogenase (NAD(P)+)], but is specific for NADP+.